regulation of myoblast fusion [GO:1901739] (biological process) Definition: Any process that modulates the frequency, rate or extent of myoblast fusion. Subtypes: GO:1901740, positive regulation of myoblast fusion [GO:1901741] References: PMID:21364645 Sources: GOC:BHF, GOC:TermGenie, GOC:rl Relationships: is a type of regulation of syncytium formation by plasma membrane fusion [GO:0060142]; regulates myoblast fusion [GO:0007520]